{
  "term_id": "GO:0045202",
  "gene": "UniProtKB:Q9Y5N1",
  "term_label": "synapse",
  "gene_symbol": "HRH3",
  "gene_name": "Histamine H3 receptor"
}